cell surface receptor signaling pathway via JAK-STAT [GO:0007259] (BP) Definition: A cell surface receptor signaling pathway in which ligand binding causes the receptor to dimerize, bringing the receptor-associated JAKs into close proximity. The JAKs then phosphorylate and activate each other on tyrosine residues.This leads to the activation of associated STAT protein, causing the STATs to dissociate from the receptor, translocate to the nucleus. The pathway ends with regulation of target gene expression by STAT proteins. References: PMID:12039028 Also known as: JAK-STAT signal transduction, receptor signaling pathway via JAK-STAT, JAK-STAT cascade Relationships: is a type of GO:0097696 Regulation: regulated by GO:0046425; negatively regulated by negative regulation of receptor signaling pathway via JAK-STAT [GO:0046426]; positively regulated by positive regulation of receptor signaling pathway via JAK-STAT [GO:0046427]